{
  "gene_symbol": "GM2A",
  "gene_name": "Ganglioside GM2 activator",
  "term_label": "cytoplasmic side of plasma membrane",
  "term_id": "GO:0009898",
  "gene": "UniProtKB:P17900"
}